{
  "term_id": "GO:0140448",
  "gene_symbol": "CSTL1",
  "term_label": "signaling receptor ligand precursor processing",
  "gene_name": "Cystatin-like 1",
  "gene": "UniProtKB:Q9H114"
}